{
  "gene_symbol": "LSR",
  "gene_name": "Lipolysis-stimulated lipoprotein receptor",
  "term_label": "tricellular tight junction assembly",
  "gene": "UniProtKB:Q86X29",
  "term_id": "GO:1904274"
}